{
  "gene_symbol": "RTF1",
  "term_label": "Unknown biological process",
  "gene_name": "RNA polymerase-associated protein RTF1 homolog",
  "term_id": "UNKNOWN:0002",
  "gene": "UniProtKB:Q92541"
}